{
  "gene": "UniProtKB:Q8IY81",
  "gene_symbol": "FTSJ3",
  "term_label": "rRNA (uridine-2'-O-)-methyltransferase activity",
  "gene_name": "pre-rRNA 2'-O-ribose RNA methyltransferase FTSJ3",
  "term_id": "GO:0008650"
}